{
  "gene": "UniProtKB:Q96CW1",
  "gene_symbol": "AP2M1",
  "term_id": "GO:0006896",
  "term_label": "Golgi to vacuole transport",
  "gene_name": "AP-2 complex subunit mu"
}